alkaloid biosynthetic process [GO:0009821] (biological process) Definition: The chemical reactions and pathways resulting in the formation of alkaloids, nitrogen-containing natural products which are not otherwise classified as nonprotein amino acids, amines, peptides, amines, cyanogenic glycosides, glucosinolates, cofactors, phytohormones, or primary metabolite (such as purine or pyrimidine bases). Sources: GOC:lr, ISBN:0122146743 Also known as: alkaloid anabolism, alkaloid biosynthesis, alkaloid formation, alkaloid synthesis Relationships: is a type of alkaloid metabolic process [GO:0009820]; is a type of GO:0044550 Subtypes: tropane alkaloid biosynthetic process [GO:0009710], GO:0009711, GO:0019503, isoquinoline alkaloid biosynthetic process [GO:0033075], indole alkaloid biosynthetic process [GO:0035835], GO:0140781, piperine biosynthetic process [GO:0160181], terrequinone A biosynthetic process [GO:1900796], pyrrolizidine alkaloid biosynthetic process [GO:1901085], nicotinate biosynthetic process [GO:1901849]